proplastid nucleoid [GO:0042647] (cellular component) Relationships: is a type of GO:0042646; is part of proplastid stroma [GO:0009571] Definition: The region of a proplastid to which the DNA is confined. Sources: GOC:jl